{
  "gene_symbol": "ZDHHC14",
  "gene": "UniProtKB:Q8IZN3",
  "term_label": "protein-cysteine S-palmitoyltransferase activity",
  "term_id": "GO:0019706",
  "gene_name": "Palmitoyltransferase ZDHHC14"
}